{
  "gene": "UniProtKB:Q9NYQ3",
  "gene_name": "2-Hydroxyacid oxidase 2",
  "term_id": "GO:0003973",
  "term_label": "(S)-2-hydroxy-acid oxidase activity",
  "gene_symbol": "HAO2"
}